{
  "gene_symbol": "DNAH11",
  "gene": "UniProtKB:Q96DT5",
  "term_label": "minus-end-directed microtubule motor activity",
  "gene_name": "Dynein axonemal heavy chain 11",
  "term_id": "GO:0008569"
}